{
  "term_id": "GO:0005634",
  "gene_name": "DNA excision repair protein ERCC-6",
  "gene": "UniProtKB:Q03468",
  "gene_symbol": "ERCC6",
  "term_label": "nucleus"
}